{
  "gene": "UniProtKB:P55157",
  "gene_name": "Microsomal triglyceride transfer protein large subunit",
  "term_id": "GO:0005783",
  "gene_symbol": "MTTP",
  "term_label": "endoplasmic reticulum"
}